{
  "gene_symbol": "CDH6",
  "gene": "UniProtKB:P55285",
  "term_id": "GO:0005912",
  "gene_name": "Cadherin-6",
  "term_label": "adherens junction"
}